head segmentation [GO:0035287] (biological process) Relationships: is a type of pattern specification process [GO:0007389]; is part of blastoderm segmentation [GO:0007350]; is part of head development [GO:0060322] Definition: Partitioning the insect head anlage into a fixed number of segmental units. The number of segments composing the insect head has long been a subject of debate, but it is generally agreed that there are 6 or 7 segments. From anterior to posterior the head segments are the procephalic segments (labral, (ocular), antennal and intercalary) and the gnathal segments (mandibular, maxillary and labial). References: PMID:10477305, PMID:7915837 Subtypes: anterior head segmentation [GO:0035288], GO:0035289 Note: See also the fly_anatomy.ontology term 'head segment ; FBbt:00000006' and its children.